{
  "gene_symbol": "SP2",
  "gene": "UniProtKB:Q02086",
  "term_id": "GO:0000978",
  "term_label": "RNA polymerase II cis-regulatory region sequence-specific DNA binding",
  "gene_name": "Transcription factor Sp2"
}